{
  "gene_symbol": "BMP4",
  "term_id": "GO:0003007",
  "gene": "UniProtKB:P12644",
  "gene_name": "Bone morphogenetic protein 4",
  "term_label": "heart morphogenesis"
}